{
  "term_label": "Unknown molecular function",
  "term_id": "UNKNOWN:0001",
  "gene_name": "Zinc finger protein 512",
  "gene": "UniProtKB:Q96ME7",
  "gene_symbol": "ZNF512"
}